{
  "term_label": "Unknown molecular function",
  "gene": "UniProtKB:Q96BM1",
  "term_id": "UNKNOWN:0001",
  "gene_symbol": "ANKRD9",
  "gene_name": "Ankyrin repeat domain-containing protein 9"
}